{
  "gene": "UniProtKB:Q9GZM6",
  "gene_symbol": "OR8D2",
  "term_label": "olfactory receptor activity",
  "gene_name": "Olfactory receptor 8D2",
  "term_id": "GO:0004984"
}